{
  "term_label": "DNA replication-dependent chromatin assembly",
  "gene_symbol": "ASF1A",
  "gene": "UniProtKB:Q9Y294",
  "gene_name": "Histone chaperone ASF1A",
  "term_id": "GO:0006335"
}